{
  "term_label": "ubiquitin protein ligase activity",
  "gene_name": "Tripartite motif-containing protein 64",
  "gene_symbol": "TRIM64",
  "gene": "UniProtKB:A6NGJ6",
  "term_id": "GO:0061630"
}